centromere separation [GO:0034510] (biological process) Subtypes: meiotic sister chromatid centromere separation [GO:0051756] Sources: GOC:mah Relationships: is a type of cell cycle process [GO:0022402]; is part of GO:0051304; is part of nuclear chromosome segregation [GO:0098813] Definition: The cell cycle process in which centromeres are physically detached from each other during chromosome separation.